{
  "gene": "UniProtKB:P0DN86",
  "gene_symbol": "CGB3",
  "term_id": "GO:0005615",
  "term_label": "extracellular space",
  "gene_name": "Choriogonadotropin subunit beta 3"
}